{
  "gene_symbol": "C5AR2",
  "term_id": "GO:0006954",
  "gene": "UniProtKB:Q9P296",
  "term_label": "inflammatory response",
  "gene_name": "C5a anaphylatoxin chemotactic receptor 2"
}